{
  "term_label": "MLL3/4 complex",
  "gene": "UniProtKB:O15054",
  "gene_symbol": "KDM6B",
  "gene_name": "Lysine-specific demethylase 6B",
  "term_id": "GO:0044666"
}